mechanosensitive voltage-gated sodium channel activity [GO:0101013] (molecular function) References: PMID:21041530, PMID:26838316 Also known as: mechanically-modulated voltage-gated sodium channel activity Definition: Enables the transmembrane transfer of a sodium ion by a voltage-gated channel whose activity is modulated in response to mechanical stress. Response to mechanical stress and voltage gating together is different than the sum of individual responses. A voltage-gated channel is a channel whose open state is dependent on the voltage across the membrane in which it is embedded. Relationships: is a type of GO:0005248; is_a GO:0140135